{
  "term_label": "translation",
  "term_id": "GO:0006412",
  "gene_name": "Large ribosomal subunit protein uL22m",
  "gene": "UniProtKB:Q9NWU5",
  "gene_symbol": "MRPL22"
}